{
  "term_label": "Unknown biological process",
  "gene_symbol": "PDC",
  "term_id": "UNKNOWN:0002",
  "gene_name": "Phosducin",
  "gene": "UniProtKB:P20941"
}